{
  "gene": "UniProtKB:Q8NEE6",
  "gene_symbol": "FBXL13",
  "gene_name": "F-box and leucine-rich repeat protein 13",
  "term_label": "SCF-dependent proteasomal ubiquitin-dependent protein catabolic process",
  "term_id": "GO:0031146"
}